{
  "term_id": "GO:0045944",
  "term_label": "positive regulation of transcription by RNA polymerase II",
  "gene_symbol": "RARG",
  "gene": "UniProtKB:P13631",
  "gene_name": "Retinoic acid receptor gamma"
}